phosphoribosylaminoimidazolecarboxamide formyltransferase activity [GO:0004643] (molecular function) Definition: Catalysis of the reaction: 10-formyltetrahydrofolate + 5'-phosphoribosyl-5-amino-4-imidazolecarboxamide = tetrahydrofolate + 5'-phosphoribosyl-5-formamido-4-imidazolecarboxamide. Sources: EC:2.1.2.3 Relationships: is a type of hydroxymethyl-, formyl- and related transferase activity [GO:0016742] Also known as: 10-formyltetrahydrofolate:5'-phosphoribosyl-5-amino-4-imidazole-carboxamide N-formyltransferase activity, 10-formyltetrahydrofolate:5'-phosphoribosyl-5-amino-4-imidazolecarboxamide formyltransferase activity, 5'-phosphoribosyl-5-amino-4-imidazolecarboxamide formyltransferase activity, 5-amino-1-ribosyl-4-imidazolecarboxamide 5'-phosphate transformylase activity, 5-amino-4-imidazolecarboxamide ribonucleotide transformylase activity, 5-amino-4-imidazolecarboxamide ribotide transformylase activity, AICAR formyltransferase activity, AICAR transformylase activity, aminoimidazolecarboxamide ribonucleotide transformylase activity